structural constituent of myelin sheath [GO:0019911] (molecular function) Sources: GOC:mah Relationships: is a type of structural molecule activity [GO:0005198]; occurs in myelin sheath [GO:0043209] Definition: The action of a molecule that contributes to the structural integrity of the myelin sheath of a nerve.